positive regulation of hormone secretion [GO:0046887] (biological process) Sources: GOC:ai Also known as: up regulation of hormone secretion, up-regulation of hormone secretion, upregulation of hormone secretion, activation of hormone secretion, stimulation of hormone secretion Definition: Any process that activates or increases the frequency, rate or extent of the regulated release of a hormone from a cell. Relationships: is_a positive regulation of cell communication [GO:0010647]; is a type of positive regulation of signaling [GO:0023056]; is a type of regulation of hormone secretion [GO:0046883]; is a type of positive regulation of secretion by cell [GO:1903532]; positively regulates hormone secretion [GO:0046879] Subtypes: positive regulation of gonadotropin secretion [GO:0032278], GO:0032337, GO:0032340, positive regulation of juvenile hormone secretion [GO:0045973], positive regulation of adiponectin secretion [GO:0070165], positive regulation of peptide hormone secretion [GO:0090277], positive regulation of histamine secretion by mast cell [GO:1903595], positive regulation of parathyroid hormone secretion [GO:2000830], positive regulation of steroid hormone secretion [GO:2000833], positive regulation of androstenedione secretion [GO:2000839], positive regulation of dehydroepiandrosterone secretion [GO:2000842], GO:2000845